{
  "term_id": "GO:0006627",
  "term_label": "protein processing involved in protein targeting to mitochondrion",
  "gene": "UniProtKB:Q10713",
  "gene_name": "Mitochondrial-processing peptidase subunit alpha",
  "gene_symbol": "PMPCA"
}